{
  "term_id": "GO:0046872",
  "gene_symbol": "MT4",
  "gene": "UniProtKB:P47944",
  "gene_name": "Metallothionein-4",
  "term_label": "metal ion binding"
}